{
  "term_id": "GO:0000070",
  "gene_name": "Protein MIS12 homolog",
  "gene": "UniProtKB:Q9H081",
  "term_label": "mitotic sister chromatid segregation",
  "gene_symbol": "MIS12"
}